{
  "gene": "UniProtKB:Q8IUB5",
  "gene_symbol": "WFDC13",
  "term_label": "extracellular space",
  "gene_name": "WAP four-disulfide core domain protein 13",
  "term_id": "GO:0005615"
}